{
  "gene": "UniProtKB:O95025",
  "gene_symbol": "SEMA3D",
  "term_id": "GO:0001755",
  "gene_name": "Semaphorin-3D",
  "term_label": "neural crest cell migration"
}